{
  "term_id": "UNKNOWN:0002",
  "gene": "UniProtKB:Q6NXN4",
  "term_label": "Unknown biological process",
  "gene_symbol": "DPY19L2P1",
  "gene_name": "Putative C-mannosyltransferase DPY19L2P1"
}